{
  "gene_name": "Coiled-coil domain-containing protein 68",
  "gene_symbol": "CCDC68",
  "term_id": "GO:0005814",
  "gene": "UniProtKB:Q9H2F9",
  "term_label": "centriole"
}